{
  "gene": "UniProtKB:Q96M93",
  "gene_symbol": "ADAD1",
  "term_label": "nucleolus",
  "gene_name": "Adenosine deaminase domain-containing protein 1",
  "term_id": "GO:0005730"
}